{
  "gene_symbol": "CASTOR1",
  "term_id": "GO:0005829",
  "gene": "UniProtKB:Q8WTX7",
  "gene_name": "Cytosolic arginine sensor for mTORC1 subunit 1",
  "term_label": "cytosol"
}